{
  "term_label": "early endosome",
  "gene_symbol": "RAB5B",
  "gene_name": "Ras-related protein Rab-5B",
  "term_id": "GO:0005769",
  "gene": "UniProtKB:P61020"
}